{
  "gene_symbol": "TRIM22",
  "term_id": "GO:0061630",
  "gene_name": "E3 ubiquitin-protein ligase TRIM22",
  "gene": "UniProtKB:Q8IYM9",
  "term_label": "ubiquitin protein ligase activity"
}